{
  "gene": "UniProtKB:Q7Z4H4",
  "gene_symbol": "ADM2",
  "term_id": "GO:0007189",
  "gene_name": "Protein ADM2",
  "term_label": "adenylate cyclase-activating G protein-coupled receptor signaling pathway"
}